{
  "term_id": "GO:0005104",
  "gene": "UniProtKB:O95750",
  "gene_name": "Fibroblast growth factor 19",
  "term_label": "fibroblast growth factor receptor binding",
  "gene_symbol": "FGF19"
}